regulation of smooth muscle contraction involved in micturition [GO:1904318] (biological process) References: PMID:18562635 Sources: GOC:TermGenie, GO_REF:0000058 Definition: Any process that modulates the frequency, rate or extent of smooth muscle contraction involved in micturition. Relationships: is a type of regulation of smooth muscle contraction [GO:0006940]; is a type of regulation of excretion [GO:0044062]; is a type of regulation of renal system process [GO:0098801]; regulates smooth muscle contraction involved in micturition [GO:0060083] Subtypes: negative regulation of smooth muscle contraction involved in micturition [GO:1904319], positive regulation of smooth muscle contraction involved in micturition [GO:1904320] Also known as: regulation of smooth muscle contraction involved in urination, regulation of urinary bladder smooth muscle contraction involved in micturition